nuclear polyadenylation-dependent CUT catabolic process [GO:0071039] (biological process) Definition: The chemical reactions and pathways occurring in the nucleus and resulting in the breakdown of a cryptic unstable transcript (CUT), initiated by the enzymatic addition of a sequence of adenylyl residues (polyadenylation) at the 3' end the target CUT. Relationships: is a type of nuclear RNA surveillance [GO:0071027]; is a type of CUT catabolic process [GO:0071034] References: PMID:15935759, PMID:16973436, PMID:16973437, PMID:18007593, PMID:18591258 Sources: GOC:dgf, GOC:krc Also known as: nuclear poly(A)-dependent CUT catabolic process